{
  "gene": "UniProtKB:P20702",
  "term_label": "integrin-mediated signaling pathway",
  "term_id": "GO:0007229",
  "gene_name": "Integrin alpha-X",
  "gene_symbol": "ITGAX"
}